transcription ternary complex [GO:0097523] (cellular component) Definition: A protein-DNA-RNA complex composed of RNA polymerase, template DNA, and an RNA transcript. Also known as: transcription protein-DNA-RNA complex Relationships: is a type of protein-DNA-RNA complex [GO:0001114] Sources: GOC:cjm, GOC:txnOH